{
  "gene": "UniProtKB:P58876",
  "gene_name": "Histone H2B type 1-D",
  "term_label": "DNA binding",
  "gene_symbol": "H2BC5",
  "term_id": "GO:0003677"
}